endopeptidase complex [GO:1905369] (cellular component) Subtypes: proteasome complex [GO:0000502], caspase complex [GO:0008303], GO:0017087, serine-type endopeptidase complex [GO:1905370], separase-securin complex [GO:1990520] Relationships: is a type of peptidase complex [GO:1905368] Note: An example of this is PLAU in human (UniProt symbol P00749) in PMID:1689240 (inferred from direct assay). References: PMID:1689240 Sources: GOC:TermGenie, GOC:bhm, GO_REF:0000088 Definition: A protein complex which is capable of endopeptidase activity.